{
  "gene": "UniProtKB:Q14141",
  "term_label": "intracellular protein localization",
  "term_id": "GO:0008104",
  "gene_symbol": "SEPTIN6",
  "gene_name": "Septin-6"
}